negative regulation of carotenoid biosynthetic process [GO:1904142] (biological process) Definition: Any process that stops, prevents or reduces the frequency, rate or extent of carotenoid biosynthetic process. References: PMID:25675505 Sources: GOC:TermGenie, GO_REF:0000058 Also known as: down regulation of carotenoid anabolism, down regulation of carotenoid biosynthesis, down regulation of carotenoid biosynthetic process, down regulation of carotenoid formation, down regulation of carotenoid synthesis, down-regulation of carotenoid anabolism, down-regulation of carotenoid biosynthesis, down-regulation of carotenoid biosynthetic process, down-regulation of carotenoid formation, down-regulation of carotenoid synthesis, downregulation of carotenoid anabolism, downregulation of carotenoid biosynthesis, downregulation of carotenoid biosynthetic process, downregulation of carotenoid formation, downregulation of carotenoid synthesis, negative regulation of carotenoid anabolism, negative regulation of carotenoid biosynthesis, negative regulation of carotenoid formation, negative regulation of carotenoid synthesis, inhibition of carotenoid anabolism, inhibition of carotenoid biosynthesis, inhibition of carotenoid biosynthetic process, inhibition of carotenoid formation, inhibition of carotenoid synthesis Relationships: is_a negative regulation of isoprenoid metabolic process [GO:0045827]; is a type of GO:0051055; negatively regulates carotenoid biosynthetic process [GO:0016117]